{
  "gene_symbol": "KRTAP4-11",
  "term_label": "Unknown molecular function",
  "gene": "UniProtKB:Q9BYQ6",
  "gene_name": "Keratin-associated protein 4-11",
  "term_id": "UNKNOWN:0001"
}